{
  "gene_symbol": "ZNF564",
  "gene_name": "Zinc finger protein 564",
  "gene": "UniProtKB:Q8TBZ8",
  "term_label": "DNA-binding transcription factor activity",
  "term_id": "GO:0003700"
}